{
  "gene_symbol": "PLD2",
  "gene": "UniProtKB:O14939",
  "gene_name": "Phospholipase D2",
  "term_id": "GO:0009395",
  "term_label": "phospholipid catabolic process"
}